{
  "gene_name": "Adhesion G protein-coupled receptor E5",
  "term_label": "G protein-coupled receptor activity",
  "gene": "UniProtKB:P48960",
  "gene_symbol": "ADGRE5",
  "term_id": "GO:0004930"
}